{
  "gene_name": "Brain acid soluble protein 1",
  "gene": "UniProtKB:P80723",
  "term_label": "transcription cis-regulatory region binding",
  "gene_symbol": "BASP1",
  "term_id": "GO:0000976"
}